{
  "term_id": "GO:2001238",
  "gene_symbol": "G0S2",
  "gene": "UniProtKB:P27469",
  "term_label": "positive regulation of extrinsic apoptotic signaling pathway",
  "gene_name": "G0_G1 switch protein 2"
}